{
  "gene": "UniProtKB:Q9BX97",
  "term_label": "regulation of vascular permeability",
  "gene_symbol": "PLVAP",
  "gene_name": "Plasmalemma vesicle-associated protein",
  "term_id": "GO:0043114"
}